sulfate adenylyltransferase (ADP) activity [GO:0004780] (molecular function) Definition: Catalysis of the reaction: ADP + H+ + sulfate = 5'-adenylyl sulfate + phosphate. Relationships: is a type of sulfate adenylyltransferase activity [GO:0004779] Also known as: ADP:sulfate adenylyltransferase activity, sulphate adenylyltransferase (ADP) activity, ADP-sulfurylase activity, adenosine diphosphate sulfurylase activity, sulfate (adenosine diphosphate) adenylyltransferase activity Sources: EC:2.7.7.5, RHEA:16529